type II interferon binding [GO:0019964] (molecular function) Relationships: is a type of interferon binding [GO:0019961] Also known as: interferon-gamma binding, IFN-gamma binding, IFNG binding Definition: Binding to type II interferon, also known as interferon-gamma. References: PMID:15546383 Sources: GOC:add, GOC:ai, ISBN:0126896631